{
  "term_id": "GO:0007268",
  "gene_symbol": "APBA2",
  "gene_name": "Amyloid-beta A4 precursor protein-binding family A member 2",
  "term_label": "chemical synaptic transmission",
  "gene": "UniProtKB:Q99767"
}